{
  "gene_symbol": "TUBE1",
  "gene_name": "Tubulin epsilon chain",
  "term_label": "microtubule",
  "gene": "UniProtKB:Q9UJT0",
  "term_id": "GO:0005874"
}